venom-mediated disruption of cell wall in another organism [GO:0044278] (biological process) References: PMID:36738900 Relationships: is a type of venom-mediated disruption of anatomical structure in another organism [GO:0140138] Definition: The disruption of the cell wall of another organism by a venom, leading to damage or temporary subversion of the cell wall. Also known as: cell wall disruption in another organism, cell wall disruption in other organism